{
  "gene_name": "Solute carrier family 26 member 9",
  "term_label": "sulfate transmembrane transport",
  "term_id": "GO:1902358",
  "gene_symbol": "SLC26A9",
  "gene": "UniProtKB:Q7LBE3"
}